{
  "gene": "UniProtKB:Q12986",
  "term_label": "RNA polymerase II transcription regulatory region sequence-specific DNA binding",
  "term_id": "GO:0000977",
  "gene_name": "Transcriptional repressor NF-X1",
  "gene_symbol": "NFX1"
}